{
  "gene": "UniProtKB:Q8IWZ8",
  "term_label": "Unknown biological process",
  "term_id": "UNKNOWN:0002",
  "gene_symbol": "SUGP1",
  "gene_name": "SURP and G-patch domain-containing protein 1"
}